{
  "term_label": "nuclear lamina",
  "term_id": "GO:0005652",
  "gene": "UniProtKB:Q03252",
  "gene_name": "Lamin-B2",
  "gene_symbol": "LMNB2"
}